{
  "gene_name": "Deoxycytidine kinase",
  "gene_symbol": "DCK",
  "gene": "UniProtKB:P27707",
  "term_label": "mitochondrion",
  "term_id": "GO:0005739"
}